{
  "gene_name": "Dermatopontin",
  "gene": "UniProtKB:Q07507",
  "term_label": "Unknown molecular function",
  "term_id": "UNKNOWN:0001",
  "gene_symbol": "DPT"
}